{
  "term_label": "Unknown biological process",
  "gene_symbol": "MRPL3",
  "gene_name": "Large ribosomal subunit protein uL3m",
  "gene": "UniProtKB:P09001",
  "term_id": "UNKNOWN:0002"
}